{
  "term_label": "postsynaptic specialization",
  "gene_name": "Disks large-associated protein 1",
  "gene": "UniProtKB:O14490",
  "gene_symbol": "DLGAP1",
  "term_id": "GO:0099572"
}